{
  "term_id": "GO:0000794",
  "gene": "UniProtKB:Q92878",
  "gene_name": "DNA repair protein RAD50",
  "term_label": "condensed nuclear chromosome",
  "gene_symbol": "RAD50"
}